{
  "term_label": "hormone activity",
  "gene_symbol": "NPPC",
  "term_id": "GO:0005179",
  "gene": "UniProtKB:P23582",
  "gene_name": "C-type natriuretic peptide"
}